{
  "term_label": "Unknown biological process",
  "gene_symbol": "TRGV2",
  "gene_name": "T cell receptor gamma variable 2",
  "gene": "UniProtKB:A0A075B6R0",
  "term_id": "UNKNOWN:0002"
}